{
  "gene_symbol": "CSNK2A2",
  "term_id": "GO:1905818",
  "gene": "UniProtKB:P19784",
  "gene_name": "Casein kinase II subunit alpha'",
  "term_label": "regulation of chromosome separation"
}